detection of hydrogen ion [GO:0003030] (biological process) Definition: The series of events in which a hydrogen ion stimulus is received by a cell and converted into a molecular signal. Subtypes: detection of pH by chemoreceptor signaling [GO:0003022] Relationships: is a type of detection of chemical stimulus [GO:0009593] Sources: GOC:mtg_cardio